{
  "gene": "UniProtKB:A8MUP2",
  "term_id": "UNKNOWN:0002",
  "term_label": "Unknown biological process",
  "gene_symbol": "CSKMT",
  "gene_name": "Citrate synthase-lysine N-methyltransferase CSKMT, mitochondrial"
}